{
  "term_label": "Unknown cellular component",
  "gene": "UniProtKB:P07099",
  "term_id": "UNKNOWN:0003",
  "gene_name": "Epoxide hydrolase 1",
  "gene_symbol": "EPHX1"
}